{
  "gene_symbol": "DHX33",
  "gene_name": "ATP-dependent RNA helicase DHX33",
  "term_id": "GO:0003725",
  "term_label": "double-stranded RNA binding",
  "gene": "UniProtKB:Q9H6R0"
}